{
  "term_label": "Unknown molecular function",
  "gene": "UniProtKB:P53814",
  "gene_name": "Smoothelin",
  "gene_symbol": "SMTN",
  "term_id": "UNKNOWN:0001"
}